{
  "gene_symbol": "VDAC2",
  "term_label": "mitochondrial outer membrane",
  "gene": "UniProtKB:P45880",
  "gene_name": "Voltage-dependent anion-selective channel protein 2",
  "term_id": "GO:0005741"
}